{
  "term_label": "cytosol",
  "term_id": "GO:0005829",
  "gene_name": "116 kDa U5 small nuclear ribonucleoprotein component",
  "gene_symbol": "EFTUD2",
  "gene": "UniProtKB:Q15029"
}